{
  "term_label": "poly(A)+ mRNA export from nucleus",
  "gene_name": "ATP-dependent RNA helicase DDX25",
  "gene_symbol": "DDX25",
  "term_id": "GO:0016973",
  "gene": "UniProtKB:Q9UHL0"
}